pyrimidodiazepine synthase activity [GO:0004734] (molecular function) Definition: Catalysis of the reaction: a pyrimidodiazepine + oxidized glutathione = 6-pyruvoyltetrahydropterin + 2 glutathione. Relationships: is a type of GO:0016648 Also known as: PDA synthase activity, pyrimidodiazepine:glutathione-disulfide oxidoreductase (ring-opening, cyclizing) Sources: EC:1.5.4.1